{
  "gene_symbol": "PIP4P2",
  "gene": "UniProtKB:Q8N4L2",
  "gene_name": "Type 2 phosphatidylinositol 4,5-bisphosphate 4-phosphatase",
  "term_label": "phosphatidylinositol dephosphorylation",
  "term_id": "GO:0046856"
}